response to amino acid [GO:0043200] (BP) Sources: GOC:ef, GOC:mlg Relationships: is a type of response to acid chemical [GO:0001101] Also known as: response to amino acid stimulus Subtypes: GO:0009961, response to proline [GO:0010238], response to L-leucine [GO:0043201], cellular response to amino acid stimulus [GO:0071230], GO:0080052, response to phenylalanine [GO:0080053], response to thyroxine [GO:0097068], response to L-thialysine [GO:1901345], response to L-canavanine [GO:1901354], response to L-cysteine [GO:1901367], response to L-glutamate [GO:1902065], response to L-arginine [GO:1903576], response to kainic acid [GO:1904373], response to L-dopa [GO:1904473], response to methionine [GO:1904640], GO:1904844, response to 3,3',5-triiodo-L-thyronine [GO:1905242], GO:1905374, response to glycine [GO:1905429] Definition: Any process that results in a change in state or activity of a cell or an organism (in terms of movement, secretion, enzyme production, gene expression, etc.) as a result of an amino acid stimulus. An amino acid is a carboxylic acids containing one or more amino groups.